15,16-dihydrobiliverdin:ferredoxin oxidoreductase activity [GO:0050617] (molecular function) Definition: Catalysis of the reaction: 15,16-dihydrobiliverdin + oxidized ferredoxin = biliverdin IXa + reduced ferredoxin. Also known as: PebA Relationships: is a type of oxidoreductase activity, acting on the CH-CH group of donors, iron-sulfur protein as acceptor [GO:0016636] Sources: EC:1.3.7.2, MetaCyc:1.3.7.2-RXN